{
  "term_id": "GO:0031841",
  "gene": "UniProtKB:P01303",
  "gene_symbol": "NPY",
  "term_label": "neuropeptide Y receptor binding",
  "gene_name": "Pro-neuropeptide Y"
}